{
  "gene_symbol": "BSN",
  "term_label": "axon",
  "gene": "UniProtKB:Q9UPA5",
  "term_id": "GO:0030424",
  "gene_name": "Protein bassoon"
}